{
  "term_label": "Unknown molecular function",
  "gene": "UniProtKB:P35443",
  "gene_name": "Thrombospondin-4",
  "gene_symbol": "THBS4",
  "term_id": "UNKNOWN:0001"
}